{
  "term_id": "GO:0043161",
  "gene": "UniProtKB:O43791",
  "term_label": "proteasome-mediated ubiquitin-dependent protein catabolic process",
  "gene_symbol": "SPOP",
  "gene_name": "Speckle-type POZ protein"
}